{
  "term_id": "GO:0045202",
  "gene": "UniProtKB:P05106",
  "gene_symbol": "ITGB3",
  "term_label": "synapse",
  "gene_name": "Integrin beta-3"
}